bacterial-type flagellum basal body [GO:0009425] (cellular component) Also known as: flagellar basal body, flagellin-based flagellum basal body Definition: One of the three major substructures of the bacterial-type flagellum, the basal body is embedded in the cell envelope (the plasma membrane, peptidoglycan cell wall, and, if one is present, the outer membrane); it houses the secretion apparatus that exports the more distal components and the flagellar motor. References: PMID:10572114, PMID:12624192, PMID:24697492 Sources: GOC:cilia, GOC:mtg_sensu Relationships: is a type of GO:0110165; is part of bacterial-type flagellum [GO:0009288]